double-stranded DNA endonuclease activity [GO:1990238] (molecular function) Subtypes: ds/ssDNA junction-specific dsDNA endonuclease activity [GO:0106332] Definition: Catalysis of the hydrolysis of ester linkages within a double-stranded DNA molecule by creating internal breaks. References: PMID:22885404 Relationships: is a type of DNA endonuclease activity [GO:0004520]; is a type of hydrolase activity, acting on ester bonds [GO:0016788] Also known as: double-stranded DNA endodeoxyribonuclease activity, dsDNA-specific endodeoxyribonuclease activity